negative regulation of biomineral tissue development [GO:0070168] (biological process) Definition: Any process that stops, prevents, or reduces the frequency, rate or extent of biomineral tissue development, the formation of hard tissues that consist mainly of inorganic compounds. Sources: GOC:mah Subtypes: negative regulation of bone mineralization [GO:0030502], negative regulation of tooth mineralization [GO:0070171], negative regulation of shell calcification [GO:1905649] Relationships: is a type of negative regulation of developmental process [GO:0051093]; is a type of regulation of biomineral tissue development [GO:0070167]; negatively regulates biomineral tissue development [GO:0031214]